{
  "term_id": "UNKNOWN:0003",
  "gene": "UniProtKB:Q5T6V5",
  "gene_symbol": "QNG1",
  "term_label": "Unknown cellular component",
  "gene_name": "Queuosine 5'-phosphate N-glycosylase_hydrolase"
}